regulation of MHC class II biosynthetic process [GO:0045346] (biological process) Subtypes: GO:0045347, GO:0045348 Also known as: regulation of MHC class II anabolism, regulation of MHC class II biosynthesis, regulation of MHC class II formation, regulation of MHC class II synthesis, regulation of major histocompatibility complex class II biosynthesis, regulation of major histocompatibility complex class II biosynthetic process Definition: Any process that modulates the frequency, rate or extent of the chemical reactions and pathways resulting in the formation of MHC class II. Sources: GOC:go_curators Relationships: is a type of regulation of macromolecule biosynthetic process [GO:0010556]; regulates MHC class II biosynthetic process [GO:0045342]